{
  "term_label": "Unknown molecular function",
  "gene": "UniProtKB:Q9Y3C1",
  "gene_name": "Nucleolar protein 16",
  "term_id": "UNKNOWN:0001",
  "gene_symbol": "NOP16"
}